positive regulation of low-density lipoprotein particle receptor catabolic process [GO:0032805] (biological process) Relationships: is a type of regulation of low-density lipoprotein particle receptor catabolic process [GO:0032803]; is a type of positive regulation of protein catabolic process [GO:0045732]; is a type of GO:2000646; positively regulates low-density lipoprotein particle receptor catabolic process [GO:0032802] Sources: GOC:mah Definition: Any process that activates or increases the frequency, rate or extent of the chemical reactions and pathways resulting in the breakdown of low-density lipoprotein particle receptors. Also known as: positive regulation of low-density lipoprotein receptor breakdown, positive regulation of low-density lipoprotein receptor catabolic process, positive regulation of low-density lipoprotein receptor catabolism, positive regulation of low-density lipoprotein receptor degradation, up regulation of low-density lipoprotein receptor catabolic process, up-regulation of low-density lipoprotein receptor catabolic process, upregulation of low-density lipoprotein receptor catabolic process, activation of low-density lipoprotein receptor catabolic process, stimulation of low-density lipoprotein receptor catabolic process